protein insertion into ER membrane by N-terminal cleaved signal sequence [GO:0045049] (biological process) Definition: A process of protein insertion into the endoplasmic reticulum (ER) membrane in which N-terminal cleaved signal sequences direct polypeptides to the ER. Relationships: is a type of protein insertion into ER membrane [GO:0045048] Also known as: N-terminal cleaved signal sequence mediated protein insertion into ER membrane, protein insertion into ER membrane, N-terminal cleaved signal sequence mediated, protein insertion into endoplasmic reticulum membrane by N-terminal cleaved signal sequence, protein-ER insertion by N-terminal cleaved signal sequence, protein-endoplasmic reticulum insertion by N-terminal cleaved signal sequence Sources: ISBN:0716731363